{
  "gene_symbol": "HOXC5",
  "term_label": "RNA polymerase II cis-regulatory region sequence-specific DNA binding",
  "gene_name": "Homeobox protein Hox-C5",
  "gene": "UniProtKB:Q00444",
  "term_id": "GO:0000978"
}